{
  "term_label": "G protein-coupled serotonin receptor activity",
  "gene_name": "5-hydroxytryptamine receptor 1A",
  "gene": "UniProtKB:P08908",
  "gene_symbol": "HTR1A",
  "term_id": "GO:0004993"
}